{
  "gene_name": "Brain-derived neurotrophic factor",
  "term_label": "extracellular space",
  "term_id": "GO:0005615",
  "gene_symbol": "BDNF",
  "gene": "UniProtKB:P23560"
}